positive regulation of mast cell activation by Fc-epsilon receptor signaling pathway [GO:0038097] (biological process) Definition: An Fc-epsilon receptor signaling pathway that results in the change in morphology and behavior of a mast cell resulting from exposure to a cytokine, chemokine, soluble factor, or to (at least in mammals) an antigen which the mast cell has specifically bound via IgE bound to Fc-epsilonRI receptors. References: PMID:12413516 Sources: GOC:phg Also known as: Fc epsilon RI-dependent mast cell activation, Fc epsilon RI-mediated mast cell activation, positive regulation of mast cell activation by Fc-epsilon receptor signalling pathway Relationships: is a type of Fc receptor mediated stimulatory signaling pathway [GO:0002431]; is_a positive regulation of mast cell activation [GO:0033005]; is a type of Fc-epsilon receptor signaling pathway [GO:0038095]